{
  "term_id": "GO:0005829",
  "gene_symbol": "AMPD3",
  "gene": "UniProtKB:Q01432",
  "term_label": "cytosol",
  "gene_name": "AMP deaminase 3"
}